maleate hydratase activity [GO:0050075] (molecular function) Also known as: (R)-malate hydro-lyase (maleate-forming), (R)-malate hydro-lyase activity, D-malate hydro-lyase activity, malease activity Relationships: is a type of hydro-lyase activity [GO:0016836] Definition: Catalysis of the reaction: (R)-malate = H2O + maleate. Sources: EC:4.2.1.31, RHEA:23692